{
  "gene": "UniProtKB:P48730",
  "term_id": "GO:0090263",
  "gene_symbol": "CSNK1D",
  "gene_name": "Casein kinase I isoform delta",
  "term_label": "positive regulation of canonical Wnt signaling pathway"
}